regulation of lysosome organization [GO:1905671] (biological process) Definition: Any process that modulates the frequency, rate or extent of lysosome organization. References: PMID:25561470 Sources: GOC:TermGenie, GO_REF:0000058 Also known as: regulation of lysosome organisation, regulation of lysosome organization and biogenesis Relationships: is a type of regulation of vacuole organization [GO:0044088]; regulates GO:0007040 Subtypes: negative regulation of lysosome organization [GO:1905672], positive regulation of lysosome organization [GO:1905673]